mitochondrial fatty acid beta-oxidation multienzyme complex [GO:0016507] (cellular component) Definition: A multienzyme complex possessing three activities in two subunits (alpha and beta) that catalyzes three steps of the fatty acid beta-oxidation cycle within the mitochondrial matrix. The alpha subunit comprises the enoyl-CoA hydratase (ECH) and 3-hydroxyacyl-CoA dehydrogenase (HACD) activities, and the beta subunit contains the acetyl-CoA C-acyltransferase (KACT)/thiolase activity. Also known as: fatty acid beta-oxidation multienzyme complex, trifunctional enzyme Relationships: is_a fatty acid beta-oxidation multienzyme complex [GO:0036125]; is a type of mitochondrial protein-containing complex [GO:0098798]; is part of mitochondrial matrix [GO:0005759] References: PMID:29915090 Sources: GOC:sjm